{
  "gene": "UniProtKB:P51668",
  "gene_name": "Ubiquitin-conjugating enzyme E2 D1",
  "term_label": "ubiquitin-dependent protein catabolic process",
  "gene_symbol": "UBE2D1",
  "term_id": "GO:0006511"
}